{
  "gene_symbol": "VPS51",
  "gene_name": "Vacuolar protein sorting-associated protein 51 homolog",
  "term_id": "GO:0048193",
  "term_label": "Golgi vesicle transport",
  "gene": "UniProtKB:Q9UID3"
}